{
  "gene_symbol": "CACNG7",
  "gene_name": "Voltage-dependent calcium channel gamma-7 subunit",
  "gene": "UniProtKB:P62955",
  "term_label": "postsynaptic neurotransmitter receptor diffusion trapping",
  "term_id": "GO:0098970"
}